{
  "gene_symbol": "CXCL12",
  "term_id": "GO:0007411",
  "term_label": "axon guidance",
  "gene_name": "Stromal cell-derived factor 1",
  "gene": "UniProtKB:P48061"
}